{
  "gene_name": "Metallothionein-1X",
  "term_label": "cytoplasm",
  "term_id": "GO:0005737",
  "gene": "UniProtKB:P80297",
  "gene_symbol": "MT1X"
}